{
  "gene_symbol": "SLC8A2",
  "gene": "UniProtKB:Q9UPR5",
  "gene_name": "Sodium_calcium exchanger 2",
  "term_id": "GO:0030424",
  "term_label": "axon"
}